{
  "gene_name": "Sulfotransferase 2B1",
  "gene": "UniProtKB:O00204",
  "term_id": "GO:0051923",
  "term_label": "sulfation",
  "gene_symbol": "SULT2B1"
}